isoorientin 3'-O-methyltransferase activity [GO:0030756] (molecular function) Also known as: S-adenosyl-L-methionine:isoorientin 3'-O-methyltransferase activity, isoorientin 3'-methyltransferase activity Definition: Catalysis of the reaction: S-adenosyl-L-methionine(1+) + isoorientin = S-adenosyl-L-homocysteine + H+ + isoscoparin. Sources: EC:2.1.1.78, RHEA:24096 Relationships: is a type of S-adenosylmethionine-dependent methyltransferase activity [GO:0008757]